{
  "gene_name": "Immunoglobulin superfamily member 10",
  "term_id": "UNKNOWN:0001",
  "gene": "UniProtKB:Q6WRI0",
  "term_label": "Unknown molecular function",
  "gene_symbol": "IGSF10"
}